{
  "term_id": "GO:0004022",
  "gene": "UniProtKB:P11766",
  "term_label": "alcohol dehydrogenase (NAD+) activity",
  "gene_symbol": "ADH5",
  "gene_name": "Alcohol dehydrogenase class-3"
}